{
  "term_label": "Unknown cellular component",
  "term_id": "UNKNOWN:0003",
  "gene": "UniProtKB:Q96JP2",
  "gene_name": "Unconventional myosin-XVB",
  "gene_symbol": "MYO15B"
}